{
  "gene_symbol": "APC2",
  "term_id": "GO:0005881",
  "gene": "UniProtKB:O95996",
  "gene_name": "Adenomatous polyposis coli protein 2",
  "term_label": "cytoplasmic microtubule"
}